RNA polymerase V complex [GO:0000419] (cellular component) Relationships: is a type of DNA-directed RNA polymerase complex [GO:0000428]; is a type of GO:0140513 Also known as: DNA-directed RNA polymerase IVb complex, DNA-directed RNA polymerase V complex References: PMID:16140984, PMID:19110459 Sources: GOC:krc, GOC:mtg_sensu Definition: RNA polymerase V is a multisubunit RNA polymerase complex found in the nucleus of plants and involved in accumulation of siRNAs and in DNA methylation-dependent silencing of endogenous repeated sequences. Pol V is composed of subunits that are paralogous or identical to the 12 subunits of Pol II. Two large subunits comprise the most conserved portion including the catalytic site and share similarity with other eukaryotic and bacterial multisubunit RNA polymerases. The second largest subunit is also found in RNA polymerase IVa, while the largest subunit is found only in the IVa complex and contains an extended C-terminal domain (CTD) that includes multiple repeats of a 16 amino-acid consensus sequence as well as other sequences. The remainder of the complex is composed of smaller subunits.